{
  "gene_name": "Eukaryotic translation initiation factor 4E transporter",
  "gene": "UniProtKB:Q9NRA8",
  "term_label": "nucleus",
  "term_id": "GO:0005634",
  "gene_symbol": "EIF4ENIF1"
}